{
  "gene": "UniProtKB:Q99551",
  "gene_name": "Transcription termination factor 1, mitochondrial",
  "term_label": "mitochondrial matrix",
  "gene_symbol": "MTERF1",
  "term_id": "GO:0005759"
}